{
  "term_label": "Unknown molecular function",
  "gene": "UniProtKB:O43586",
  "gene_symbol": "PSTPIP1",
  "gene_name": "Proline-serine-threonine phosphatase-interacting protein 1",
  "term_id": "UNKNOWN:0001"
}